protein uridylylation [GO:0018177] (biological process) Subtypes: peptidyl-histidine uridylylation [GO:0051114] Sources: GOC:jsg Also known as: protein amino acid uridylylation Relationships: is a type of protein nucleotidylation [GO:0018175] Definition: The addition of phospho-uridine to a protein amino acid.